{
  "term_label": "Golgi apparatus",
  "gene_symbol": "SLC35D1",
  "gene": "UniProtKB:Q9NTN3",
  "term_id": "GO:0005794",
  "gene_name": "Nucleotide sugar transporter SLC35D1"
}